{
  "term_id": "UNKNOWN:0002",
  "gene": "UniProtKB:Q6ZUI0",
  "gene_name": "Tumor protein p63-regulated gene 1 protein",
  "gene_symbol": "TPRG1",
  "term_label": "Unknown biological process"
}